symbiont entry into host cell via disruption of host cell glycocalyx [GO:0098996] (biological process) Also known as: catabolism of host glycocalyx during viral entry, degradation of host capsule during virus entry, degradation of host glycocalyx during viral entry, disassembly of glycocalyx during viral entry, disruption of host cell glycocalyx during viral entry, symbiont entry into host cell by disruption of host cell capsule Sources: GOC:dos Definition: The disruption by a symbiont of host cell capsule to allow entry into the host cell. Relationships: is a type of symbiont-mediated disruption of host cell envelope [GO:0098933]; is part of symbiont entry into host cell [GO:0046718]